{
  "gene_symbol": "SLC8A1",
  "term_id": "GO:0035725",
  "term_label": "sodium ion transmembrane transport",
  "gene_name": "Sodium_calcium exchanger 1",
  "gene": "UniProtKB:P32418"
}